cobalamin biosynthetic process [GO:0009236] (biological process) Definition: The chemical reactions and pathways resulting in the formation of cobalamin (vitamin B12), a water-soluble vitamin characterized by possession of a corrin nucleus containing a cobalt atom. Relationships: is a type of GO:0009235; is a type of tetrapyrrole biosynthetic process [GO:0033014]; is_a water-soluble vitamin biosynthetic process [GO:0042364] Also known as: cobalamin anabolism, cobalamin biosynthesis, cobalamin formation, cobalamin synthesis, vitamin B12 biosynthesis, vitamin B12 biosynthetic process Subtypes: aerobic cobalamin biosynthetic process [GO:0019250], anaerobic cobalamin biosynthetic process [GO:0019251] Sources: GOC:jl, ISBN:0198506732